{
  "term_label": "mitochondrial matrix",
  "gene": "UniProtKB:O95900",
  "gene_name": "Pseudouridylate synthase TRUB2, mitochondrial",
  "gene_symbol": "TRUB2",
  "term_id": "GO:0005759"
}